{
  "term_id": "GO:0048471",
  "term_label": "perinuclear region of cytoplasm",
  "gene_name": "Endoplasmin",
  "gene": "UniProtKB:P14625",
  "gene_symbol": "HSP90B1"
}